{
  "gene": "UniProtKB:O75912",
  "term_id": "GO:0006654",
  "gene_symbol": "DGKI",
  "term_label": "phosphatidic acid biosynthetic process",
  "gene_name": "Diacylglycerol kinase iota"
}